{
  "term_label": "Unknown cellular component",
  "gene_name": "Immunoglobulin heavy variable 3_OR16-9 (non-functional) (Fragment)",
  "term_id": "UNKNOWN:0003",
  "gene": "UniProtKB:A0A0B4J2B5",
  "gene_symbol": "IGHV3OR16-9"
}